{
  "gene_symbol": "MAGEB6",
  "term_label": "Unknown molecular function",
  "gene_name": "Melanoma-associated antigen B6",
  "gene": "UniProtKB:Q8N7X4",
  "term_id": "UNKNOWN:0001"
}